positive regulation of capsule polysaccharide biosynthetic process [GO:0062085] (biological process) Definition: Any process that activates, maintains or increases the frequency, rate or extent of the chemical reactions and pathways resulting in the formation of polysaccharides that make up the capsule, a protective structure surrounding some species of bacteria and fungi. Relationships: is a type of positive regulation of macromolecule biosynthetic process [GO:0010557]; is a type of positive regulation of carbohydrate metabolic process [GO:0045913]; is a type of regulation of capsule polysaccharide biosynthetic process [GO:0062084]; is a type of positive regulation of capsule organization [GO:1901915]; positively regulates capsule polysaccharide biosynthetic process [GO:0045227] References: PMID:21917918